{
  "gene": "UniProtKB:Q9H2U2",
  "gene_symbol": "PPA2",
  "gene_name": "Inorganic pyrophosphatase 2, mitochondrial",
  "term_id": "GO:0006796",
  "term_label": "phosphate-containing compound metabolic process"
}